acyl-[acyl-carrier-protein]-phospholipid O-acyltransferase activity [GO:0008779] (molecular function) Also known as: acyl-ACP-phospholipid O-acyltransferase activity, acyl-[acyl-carrier protein]-phospholipid O-acyltransferase activity, acyl-acyl-carrier-protein-phospholipid O-acyltransferase activity, acyl-acyl-carrier-protein:O-(2-acyl-sn-glycero-3-phospho)-ethanolamine O-acyltransferase activity Definition: Catalysis of the reaction: acyl-[acyl-carrier protein] + O-(2-acyl-sn-glycero-3-phospho)ethanolamine = [acyl-carrier protein] + O-(1-beta-acyl-2-acyl-sn-glycero-3-phospho)ethanolamine. Relationships: is a type of O-acyltransferase activity [GO:0008374] Sources: EC:2.3.1.40